{
  "gene_symbol": "SOWAHC",
  "term_label": "Unknown molecular function",
  "gene": "UniProtKB:Q53LP3",
  "term_id": "UNKNOWN:0001",
  "gene_name": "Ankyrin repeat domain-containing protein SOWAHC"
}